{
  "gene_name": "Protein TESPA1",
  "term_label": "positive regulation of T cell receptor signaling pathway",
  "term_id": "GO:0050862",
  "gene": "UniProtKB:A2RU30",
  "gene_symbol": "TESPA1"
}